regulation of triglyceride catabolic process [GO:0010896] (biological process) Definition: Any process that modulates the frequency, rate, or extent of the chemical reactions and pathways resulting in the breakdown of triglyceride. Subtypes: negative regulation of triglyceride catabolic process [GO:0010897], GO:0010898 Sources: GOC:rn, GOC:tb Also known as: regulation of triacylglycerol catabolic process Relationships: is a type of regulation of lipid catabolic process [GO:0050994]; is a type of regulation of triglyceride metabolic process [GO:0090207]; regulates triglyceride catabolic process [GO:0019433]